oxidoreductase activity, acting on a sulfur group of donors, quinone or similar compound as acceptor [GO:0016672] (molecular function) Subtypes: thiosulfate dehydrogenase (quinone) activity [GO:0043831], GO:0045174, GO:0070224, glutathione-dependent sulfide quinone oxidoreductase activity [GO:0106436] Sources: GOC:jl Definition: Catalysis of an oxidation-reduction (redox) reaction in which a sulfur-containing group acts as a hydrogen or electron donor and reduces quinone or a related compound. Also known as: oxidoreductase activity, acting on sulphur group of donors, quinone or similar compound as acceptor Relationships: is a type of GO:0016667